{
  "gene": "UniProtKB:Q96FJ2",
  "term_id": "GO:0005868",
  "gene_symbol": "DYNLL2",
  "gene_name": "Dynein light chain 2, cytoplasmic",
  "term_label": "cytoplasmic dynein complex"
}